synaptic vesicle membrane [GO:0030672] (cellular component) Sources: GOC:mah Definition: The lipid bilayer surrounding a synaptic vesicle. Relationships: is_a exocytic vesicle membrane [GO:0099501]; is part of synaptic vesicle [GO:0008021]